{
  "term_id": "UNKNOWN:0003",
  "gene_symbol": "A0A804HJP8",
  "gene_name": "Uncharacterized protein",
  "term_label": "Unknown cellular component",
  "gene": "UniProtKB:A0A804HJP8"
}